{
  "term_id": "GO:0008017",
  "term_label": "microtubule binding",
  "gene": "UniProtKB:Q6ZUX3",
  "gene_symbol": "TOGARAM2",
  "gene_name": "TOG array regulator of axonemal microtubules protein 2"
}